{
  "gene": "UniProtKB:Q7Z6A9",
  "gene_symbol": "BTLA",
  "gene_name": "B- and T-lymphocyte attenuator",
  "term_id": "GO:0002768",
  "term_label": "immune response-regulating cell surface receptor signaling pathway"
}